active transmembrane transporter activity [GO:0022804] (molecular function) Sources: GOC:mtg_transport, ISBN:0815340729 Definition: Enables the transfer of a specific substance or related group of substances from one side of a membrane to the other, up the solute's concentration gradient. The transporter binds the solute and undergoes a series of conformational changes. Transport works equally well in either direction. Relationships: is a type of GO:0022857 Also known as: active carrier activity, carrier activity, permease activity, pump activity Subtypes: GO:0008504, GO:0008982, secondary active transmembrane transporter activity [GO:0015291], primary active transmembrane transporter activity [GO:0015399], sorbitol transmembrane transporter activity [GO:0015576], active borate transmembrane transporter activity [GO:0046715], protein-phosphocysteine-sugar phosphotransferase activity [GO:0090563]